{
  "gene_name": "Sodium-coupled neutral amino acid symporter 1",
  "term_id": "GO:0005886",
  "gene": "UniProtKB:Q9H2H9",
  "term_label": "plasma membrane",
  "gene_symbol": "SLC38A1"
}